{
  "term_label": "Unknown biological process",
  "term_id": "UNKNOWN:0002",
  "gene_symbol": "PDE6D",
  "gene": "UniProtKB:O43924",
  "gene_name": "Retinal rod rhodopsin-sensitive cGMP 3',5'-cyclic phosphodiesterase subunit delta"
}